{
  "term_id": "GO:0005886",
  "gene": "UniProtKB:Q9BRI3",
  "gene_symbol": "SLC30A2",
  "gene_name": "Proton-coupled zinc antiporter SLC30A2",
  "term_label": "plasma membrane"
}